{
  "gene_symbol": "DLC1",
  "term_id": "GO:0005925",
  "term_label": "focal adhesion",
  "gene_name": "Rho GTPase-activating protein 7",
  "gene": "UniProtKB:Q96QB1"
}